{
  "gene_name": "Proteasome subunit alpha type-6",
  "term_label": "proteasome-mediated ubiquitin-dependent protein catabolic process",
  "term_id": "GO:0043161",
  "gene_symbol": "PSMA6",
  "gene": "UniProtKB:P60900"
}